cannabidiolate synthase activity [GO:0102779] (molecular function) Sources: GOC:pz, RHEA:34411 Relationships: is a type of GO:0046993 Definition: Catalysis of the reaction: cannabigerolate + O2 = cannabidiolate + hydrogen peroxide.